D-glutamate cyclase activity [GO:0047820] (molecular function) Relationships: is a type of cyclase activity [GO:0009975]; is a type of hydro-lyase activity [GO:0016836] Sources: RHEA:22360 Also known as: D-glutamate hydro-lyase (cyclizing), D-glutamate hydro-lyase (cyclizing; 5-oxo-D-proline-forming) Definition: Catalysis of the reaction: D-glutamate = 5-oxo-D-proline + H2O.